{
  "gene_name": "Protein FAM227A",
  "gene": "UniProtKB:F5H4B4",
  "gene_symbol": "FAM227A",
  "term_label": "Unknown molecular function",
  "term_id": "UNKNOWN:0001"
}